{
  "gene_symbol": "LPP",
  "term_label": "Unknown molecular function",
  "gene_name": "Lipoma-preferred partner",
  "term_id": "UNKNOWN:0001",
  "gene": "UniProtKB:Q93052"
}